{
  "term_label": "Unknown molecular function",
  "gene_name": "Putative uncharacterized protein encoded by LINC00052",
  "term_id": "UNKNOWN:0001",
  "gene_symbol": "LINC00052",
  "gene": "UniProtKB:Q96N35"
}